regulation of pollen tube growth [GO:0080092] (biological process) Relationships: is a type of regulation of multicellular organismal process [GO:0051239]; is_a GO:0051510; is a type of GO:2000241; regulates GO:0009860 References: PMID:19208902 Definition: Any process that modulates the frequency, rate or extent of pollen tube growth.